{
  "term_label": "Unknown biological process",
  "gene": "UniProtKB:Q4VC44",
  "gene_symbol": "FLYWCH1",
  "gene_name": "FLYWCH-type zinc finger-containing protein 1",
  "term_id": "UNKNOWN:0002"
}